{
  "term_label": "mitochondrial respirasome assembly",
  "gene_name": "HIG1 domain family member 1A, mitochondrial",
  "gene": "UniProtKB:Q9Y241",
  "term_id": "GO:0097250",
  "gene_symbol": "HIGD1A"
}